{
  "gene_symbol": "CLUHP3",
  "term_label": "Unknown cellular component",
  "gene": "UniProtKB:Q96NS8",
  "gene_name": "Putative protein CLUHP3",
  "term_id": "UNKNOWN:0003"
}